{
  "gene": "UniProtKB:Q9UBX1",
  "term_id": "GO:0004197",
  "gene_name": "Cathepsin F",
  "term_label": "cysteine-type endopeptidase activity",
  "gene_symbol": "CTSF"
}